{
  "term_label": "Golgi transport complex",
  "gene_name": "Conserved oligomeric Golgi complex subunit 6",
  "term_id": "GO:0017119",
  "gene_symbol": "COG6",
  "gene": "UniProtKB:Q9Y2V7"
}